positive regulation of the force of heart contraction by circulating epinephrine [GO:0003088] (biological process) Relationships: is a type of GO:0003059; is part of positive regulation of the force of heart contraction by circulating epinephrine-norepinephrine [GO:0003089] Definition: The process in which the secretion of epinephrine into the bloodstream modulates the force of heart muscle contraction. Also known as: increased force of heart contraction by epinephrine in the bloodstream, increased force of heart contraction by circulating adrenaline, positive regulation of heart contraction by circulating adrenaline, positive regulation of heart contraction by circulating epinephrine Sources: GOC:mtg_cardio